{
  "term_id": "UNKNOWN:0002",
  "gene": "UniProtKB:P78524",
  "term_label": "Unknown biological process",
  "gene_symbol": "DENND2B",
  "gene_name": "DENN domain-containing protein 2B"
}